{
  "term_label": "regulation of transcription by RNA polymerase II",
  "term_id": "GO:0006357",
  "gene_symbol": "ZNF829",
  "gene": "UniProtKB:Q3KNS6",
  "gene_name": "Zinc finger protein 829"
}